{
  "gene_name": "General transcription and DNA repair factor IIH helicase subunit XPB",
  "term_label": "nucleotide-excision repair factor 3 complex",
  "gene": "UniProtKB:P19447",
  "gene_symbol": "ERCC3",
  "term_id": "GO:0000112"
}